{
  "gene": "UniProtKB:Q96H72",
  "term_label": "Unknown cellular component",
  "term_id": "UNKNOWN:0003",
  "gene_symbol": "SLC39A13",
  "gene_name": "Zinc transporter ZIP13"
}